phosphoenolpyruvate-protein phosphotransferase activity [GO:0008965] (molecular function) Definition: Catalysis of the reaction: phosphoenolpyruvate + protein L-histidine = pyruvate + protein N(pi)-phospho-L-histidine. Also known as: enzyme I of the phosphotransferase system, sugar--PEP phosphotransferase enzyme I activity, phosphoenolpyruvate sugar phosphotransferase enzyme I activity, phosphoenolpyruvate--protein phosphatase activity, phosphoenolpyruvate:protein-L-histidine N-pros-phosphotransferase activity, phosphoenolpyruvate:protein-L-histidine Npi-phosphotransferase activity, phosphopyruvate--protein factor phosphotransferase activity, phosphopyruvate--protein phosphotransferase activity Relationships: is a type of phosphotransferase activity, nitrogenous group as acceptor [GO:0016775] Sources: EC:2.7.3.9